{
  "term_id": "GO:0006096",
  "gene": "UniProtKB:P35557",
  "term_label": "glycolytic process",
  "gene_symbol": "GCK",
  "gene_name": "Hexokinase-4"
}